{
  "gene_name": "ATP-binding cassette sub-family D member 2",
  "term_label": "ATPase-coupled transmembrane transporter activity",
  "gene": "UniProtKB:Q9UBJ2",
  "gene_symbol": "ABCD2",
  "term_id": "GO:0042626"
}